{
  "term_id": "GO:0004867",
  "gene_symbol": "WFDC2",
  "gene": "UniProtKB:Q14508",
  "term_label": "serine-type endopeptidase inhibitor activity",
  "gene_name": "WAP four-disulfide core domain protein 2"
}